methylquinoline catabolic process [GO:0019335] (biological process) Relationships: is a type of xenobiotic catabolic process [GO:0042178] Definition: The chemical reactions and pathways resulting in the breakdown of methylquinoline, an aromatic compound composed of a benzene ring and a heterocyclic N-containing ring. References: PMID:10746195 Sources: GOC:ai Also known as: 2-methylquinoline catabolic process, 3-methylquinoline breakdown, 3-methylquinoline catabolic process, 3-methylquinoline catabolism, 3-methylquinoline degradation, quinaldine catabolic process